{
  "term_id": "GO:0016020",
  "gene": "UniProtKB:Q9BRQ5",
  "term_label": "membrane",
  "gene_name": "Protein orai-3",
  "gene_symbol": "ORAI3"
}